sensory perception of gravity [GO:0070998] (biological process) Sources: GOC:mah Relationships: is a type of GO:0007600 Definition: The series of events required for an organism to receive a gravitational stimulus, convert it to a molecular signal, and recognize and characterize the signal. This is a neurological process.